{
  "term_id": "GO:0019770",
  "gene": "UniProtKB:O75015",
  "term_label": "IgG receptor activity",
  "gene_symbol": "FCGR3B",
  "gene_name": "Low affinity immunoglobulin gamma Fc region receptor III-B"
}